male germ-line cyst encapsulation [GO:0048140] (biological process) Definition: Formation of a single follicular epithelium around the germ-line derived cells of a cyst formed in the male gonad. References: PMID:11591336 Sources: GOC:jid Relationships: is a type of germ-line cyst encapsulation [GO:0048138]; is part of spermatogenesis [GO:0007283]